{
  "gene_symbol": "RSKR",
  "term_label": "Unknown biological process",
  "gene": "UniProtKB:Q96LW2",
  "gene_name": "Ribosomal protein S6 kinase-related protein",
  "term_id": "UNKNOWN:0002"
}